regulation of ecdysteroid metabolic process [GO:0007553] (biological process) Also known as: regulation of ecdysteroid metabolism Definition: Any process that modulates the frequency, rate or extent of the chemical reactions and pathways involving ecdysteroids, a group of polyhydroxylated ketosteroids which initiate post-embryonic development, including the metamorphosis of immature forms and the development of the reproductive system and the maturation of oocytes in adult females. Relationships: is a type of regulation of ketone metabolic process [GO:0010565]; is a type of regulation of steroid metabolic process [GO:0019218]; is a type of GO:0032350; regulates ecdysteroid metabolic process [GO:0045455] Sources: ISBN:0198506732 Subtypes: regulation of ecdysteroid biosynthetic process [GO:0007554]